acetyl-CoA C-acyltransferase activity [GO:0003988] (molecular function) Relationships: is a type of C-acyltransferase activity [GO:0016408] Sources: RHEA:21564 Also known as: 2-keto-acyl thiolase activity, 3-ketoacyl coenzyme A thiolase activity, 3-ketoacyl-CoA thiolase activity, 3-ketothiolase activity, acetoacetyl-CoA beta-ketothiolase activity, acetyl-CoA acyltransferase activity, beta-ketoacyl coenzyme A thiolase activity, beta-ketothiolase activity Definition: Catalysis of the reaction: acyl-CoA + acetyl-CoA = CoA + 3-oxoacyl-CoA. Subtypes: GO:0003985, 3-oxoadipyl-CoA thiolase activity [GO:0033812]